{
  "term_id": "GO:0007417",
  "term_label": "central nervous system development",
  "gene_name": "Transcription factor SOX-6",
  "gene_symbol": "SOX6",
  "gene": "UniProtKB:P35712"
}